{
  "gene_symbol": "OPN1MW3",
  "gene": "UniProtKB:P0DN78",
  "term_label": "G protein-coupled photoreceptor activity",
  "term_id": "GO:0008020",
  "gene_name": "Medium-wave-sensitive opsin 3"
}